{
  "gene_symbol": "ACP4",
  "gene_name": "Testicular acid phosphatase",
  "term_label": "acid phosphatase activity",
  "gene": "UniProtKB:Q9BZG2",
  "term_id": "GO:0003993"
}